{
  "gene": "UniProtKB:Q8WWR8",
  "term_id": "GO:0006689",
  "gene_name": "Sialidase-4",
  "gene_symbol": "NEU4",
  "term_label": "ganglioside catabolic process"
}